{
  "gene_name": "Beta-parvin",
  "term_id": "GO:0030027",
  "gene": "UniProtKB:Q9HBI1",
  "term_label": "lamellipodium",
  "gene_symbol": "PARVB"
}